calcium/calmodulin-dependent protein kinase activity [GO:0004683] (molecular function) References: PMID:11264466 Sources: GOC:mah Definition: Calmodulin-dependent catalysis of the reactions: ATP + a protein serine = ADP + protein serine phosphate; and ATP + a protein threonine = ADP + protein threonine phosphate. This activity require the presence of calcium-bound calmodulin. Subtypes: elongation factor-2 kinase activity [GO:0004686], phosphorylase kinase activity [GO:0004689], myosin heavy chain kinase activity [GO:0016905] Also known as: Ca2+/CaM-dependent kinase activity, calcium- and calmodulin-dependent protein kinase activity, calmodulin regulated protein kinase activity, calmodulin-dependent protein kinase activity, ATP:caldesmon O-phosphotransferase activity, Ca2+/calmodulin-dependent microtubule-associated protein 2 kinase activity, Ca2+/calmodulin-dependent protein kinase 1 activity, Ca2+/calmodulin-dependent protein kinase II activity, Ca2+/calmodulin-dependent protein kinase IV activity, Ca2+/calmodulin-dependent protein kinase kinase activity, Ca2+/calmodulin-dependent protein kinase kinase beta activity, CaM kinase II activity, calcium/calmodulin-dependent protein kinase type II activity, caldesmon kinase (phosphorylating) activity, calmodulin-dependent kinase II activity, calmodulin-dependent protein kinase I activity, ATP:protein phosphotransferase (Ca2+/calmodulin-dependent) activity, CAM PKII, Ca2+/calmodulin-dependent protein kinase activity, CaM kinase activity, CaM-regulated serine/threonine kinase activity, CaMKI, CaMKII, CaMKIV, CaMKKalpha, CaMKKbeta, STK20, microtubule-associated protein 2 kinase activity, multifunctional calcium- and calmodulin-regulated protein kinase activity, multifunctional calcium/calmodulin regulated protein kinase activity Relationships: is a type of protein serine/threonine kinase activity [GO:0004674]